forebrain generation of neurons [GO:0021872] (biological process) Also known as: generation of neurons in forebrain Sources: GOC:cls, GOC:dgh, GOC:dph, GOC:jid, GO_REF:0000021 Relationships: is a type of generation of neurons [GO:0048699]; BFO_0000050 GO:0030900 Definition: The process in which nerve cells are generated in the forebrain. This includes the production of neuroblasts from and their differentiation into neurons.